positive regulation of T cell tolerance induction to tumor cell [GO:0002848] (biological process) Definition: Any process that activates or increases the frequency, rate, or extent of T cell tolerance induction to tumor cell. Sources: GOC:add Relationships: is a type of positive regulation of T cell mediated immune response to tumor cell [GO:0002842]; is_a positive regulation of tolerance induction to tumor cell [GO:0002845]; is a type of regulation of T cell tolerance induction to tumor cell [GO:0002846]; is_a positive regulation of peripheral T cell tolerance induction [GO:0002851]; positively regulates T cell tolerance induction to tumor cell [GO:0002411] Also known as: up regulation of T cell tolerance induction to tumor cell, up-regulation of T cell tolerance induction to tumor cell, upregulation of T cell tolerance induction to tumor cell, activation of T cell tolerance induction to tumor cell, stimulation of T cell tolerance induction to tumor cell